{
  "gene_name": "SERTA domain-containing protein 1",
  "gene_symbol": "SERTAD1",
  "term_label": "nucleus",
  "gene": "UniProtKB:Q9UHV2",
  "term_id": "GO:0005634"
}